I band [GO:0031674] (cellular component) Also known as: I disc, J disc, isotropic disc Sources: ISBN:0321204131 Relationships: is a type of GO:0110165; is part of sarcomere [GO:0030017] Definition: A region of a sarcomere that appears as a light band on each side of the Z disc, comprising a region of the sarcomere where thin (actin) filaments are not overlapped by thick (myosin) filaments; contains actin, troponin, and tropomyosin; each sarcomere includes half of an I band at each end.